{
  "gene_name": "Zona pellucida-binding protein 1",
  "term_label": "acrosome assembly",
  "gene_symbol": "ZPBP",
  "gene": "UniProtKB:Q9BS86",
  "term_id": "GO:0001675"
}